{
  "gene_symbol": "PTP4A3",
  "gene_name": "Protein tyrosine phosphatase type IVA 3",
  "gene": "UniProtKB:O75365",
  "term_id": "GO:0043542",
  "term_label": "endothelial cell migration"
}